{
  "gene_name": "Cadherin-7",
  "gene": "UniProtKB:Q9ULB5",
  "term_id": "GO:0044331",
  "gene_symbol": "CDH7",
  "term_label": "cell-cell adhesion mediated by cadherin"
}